positive regulation of oligodendrocyte apoptotic process [GO:1900143] (biological process) Sources: GOC:TermGenie, GOC:yaf Definition: Any process that activates or increases the frequency, rate or extent of oligodendrocyte apoptotic process. Relationships: is a type of positive regulation of glial cell apoptotic process [GO:0034352]; is a type of GO:1900141; positively regulates oligodendrocyte apoptotic process [GO:0097252] Also known as: up regulation of oligodendrocyte apoptotic process, up-regulation of oligodendrocyte apoptotic process, upregulation of oligodendrocyte apoptotic process, activation of oligodendrocyte apoptosis, activation of oligodendrocyte apoptotic process, positive regulation of oligodendrocyte apoptosis, up regulation of oligodendrocyte apoptosis, up-regulation of oligodendrocyte apoptosis, upregulation of oligodendrocyte apoptosis